{
  "term_label": "Ras protein signal transduction",
  "gene_name": "Ral guanine nucleotide dissociation stimulator",
  "gene": "UniProtKB:Q12967",
  "term_id": "GO:0007265",
  "gene_symbol": "RALGDS"
}